{
  "gene_symbol": "EXOSC10",
  "term_id": "GO:0000467",
  "term_label": "exonucleolytic trimming to generate mature 3'-end of 5.8S rRNA from tricistronic rRNA transcript (SSU-rRNA, 5.8S rRNA, LSU-rRNA)",
  "gene": "UniProtKB:Q01780",
  "gene_name": "Exosome component 10"
}